DNA-dependent protein kinase complex [GO:0070418] (cellular component) References: PMID:10854421, PMID:12235392 Sources: GOC:mah Also known as: DNA-PK complex, DNA-PK-Ku antigen complex, DNA-dependent protein kinase, DNA-end-binding complex Relationships: is a type of nuclear protein-containing complex [GO:0140513]; is a type of serine/threonine protein kinase complex [GO:1902554] Definition: A protein complex that is involved in the repair of DNA double-strand breaks and, in mammals, V(D)J recombination events. It consists of the DNA-dependent protein kinase catalytic subunit (DNA-PKcs) and the DNA end-binding heterodimer Ku.